ATP-activated inward rectifier potassium channel activity [GO:0015272] (molecular function) Definition: Enables the transmembrane transfer of a potassium ion by an inwardly-rectifying voltage-gated channel, where the inward rectification is due to a voltage-dependent block of the channel pore by ATP. An inwardly rectifying current-voltage relation is one where at any given driving force the inward flow of K+ ions exceeds the outward flow for the opposite driving force. Sources: GOC:cb, GOC:mah Relationships: is a type of GO:0005242